{
  "term_id": "GO:0005634",
  "gene_symbol": "ARRB1",
  "gene_name": "Beta-arrestin-1",
  "term_label": "nucleus",
  "gene": "UniProtKB:P49407"
}